{
  "gene_symbol": "PARP9",
  "term_label": "nucleus",
  "term_id": "GO:0005634",
  "gene_name": "Protein mono-ADP-ribosyltransferase PARP9",
  "gene": "UniProtKB:Q8IXQ6"
}